negative regulation of ectodermal cell fate specification [GO:0042666] (biological process) Definition: Any process that restricts, stops or prevents a cell from specifying into an ectoderm cell. Sources: GOC:go_curators Relationships: is a type of negative regulation of cell fate specification [GO:0009996]; is_a regulation of ectodermal cell fate specification [GO:0042665]; negatively regulates GO:0001715 Also known as: down regulation of ectodermal cell fate specification, down-regulation of ectodermal cell fate specification, downregulation of ectodermal cell fate specification, negative regulation of ectoderm cell fate specification, suppression of ectoderm cell fate, suppression of ectodermal cell fate, inhibition of ectodermal cell fate specification